{
  "gene": "UniProtKB:P33241",
  "gene_symbol": "LSP1",
  "gene_name": "Lymphocyte-specific protein 1",
  "term_id": "UNKNOWN:0003",
  "term_label": "Unknown cellular component"
}